synergid differentiation [GO:0009563] (biological process) Sources: GOC:jid Relationships: is a type of cell differentiation [GO:0030154]; is part of megagametogenesis [GO:0009561] Definition: The process in which an uncellularized nucleus cellularizes and acquires the specialized features of a synergid cell. Regulation: regulated by GO:0045697; negatively regulated by negative regulation of synergid differentiation [GO:0045698]; RO_0002213 by positive regulation of synergid differentiation [GO:0045699] Also known as: synergid cell differentiation